{
  "gene_name": "Putative cytosolic acyl coenzyme A thioester hydrolase-like",
  "term_id": "GO:0005737",
  "term_label": "cytoplasm",
  "gene_symbol": "ACOT7L",
  "gene": "UniProtKB:Q6ZUV0"
}